{
  "gene_name": "V-type immunoglobulin domain-containing suppressor of T-cell activation",
  "term_label": "negative regulation of alpha-beta T cell activation",
  "term_id": "GO:0046636",
  "gene": "UniProtKB:Q9H7M9",
  "gene_symbol": "VSIR"
}